negative regulation of cell population proliferation [GO:0008285] (biological process) Relationships: is a type of GO:0042127; is a type of GO:0048523; negatively regulates cell population proliferation [GO:0008283] Also known as: down regulation of cell proliferation, down-regulation of cell proliferation, downregulation of cell proliferation, inhibition of cell proliferation, negative regulation of cell proliferation Sources: GOC:go_curators Subtypes: negative regulation of skeletal muscle cell proliferation [GO:0014859], negative regulation of osteoblast proliferation [GO:0033689], GO:0035207, negative regulation of fibroblast proliferation [GO:0048147], negative regulation of smooth muscle cell proliferation [GO:0048662], GO:0050680, GO:0060044, negative regulation of cell proliferation involved in contact inhibition [GO:0060244], negative regulation of glial cell proliferation [GO:0060253], negative regulation of growth plate cartilage chondrocyte proliferation [GO:0061914], negative regulation of fat cell proliferation [GO:0070345], negative regulation of leukocyte proliferation [GO:0070664], negative regulation of hair follicle cell proliferation [GO:0071337], negative regulation of mesenchymal cell proliferation [GO:0072201], GO:1901383, negative regulation of cell proliferation involved in kidney development [GO:1901723], negative regulation of chondrocyte proliferation [GO:1902731], negative regulation of cell proliferation in bone marrow [GO:1903769], negative regulation of trophectodermal cell proliferation [GO:1904074], GO:1905937, negative regulation of mammary stem cell proliferation [GO:2000102], negative regulation of cell proliferation involved in heart morphogenesis [GO:2000137], GO:2000178, negative regulation of cell proliferation involved in compound eye morphogenesis [GO:2000496], negative regulation of stem cell proliferation [GO:2000647], negative regulation of myoblast proliferation [GO:2000818] Definition: Any process that stops, prevents or reduces the rate or extent of cell proliferation.